{
  "gene_name": "Gamma-aminobutyric acid receptor subunit beta-3",
  "term_label": "chloride transmembrane transport",
  "gene_symbol": "GABRB3",
  "term_id": "GO:1902476",
  "gene": "UniProtKB:P28472"
}